regulation of membrane repolarization [GO:0060306] (biological process) Relationships: is a type of regulation of membrane potential [GO:0042391]; is a type of regulation of biological process [GO:0050789]; regulates membrane repolarization [GO:0086009] Definition: Any process that modulates the establishment or extent of a membrane potential in the polarizing direction towards the resting potential, usually from positive to negative. Sources: GOC:BHF, GOC:dph, GOC:mtg_cardiac_conduct_nov11, GOC:tb Subtypes: regulation of membrane repolarization during action potential [GO:0098903], GO:0099623